{
  "gene": "UniProtKB:Q13563",
  "term_id": "GO:0051209",
  "term_label": "release of sequestered calcium ion into cytosol",
  "gene_symbol": "PKD2",
  "gene_name": "Polycystin-2"
}